{
  "gene": "UniProtKB:Q8TDY2",
  "term_label": "reticulophagy",
  "term_id": "GO:0061709",
  "gene_symbol": "RB1CC1",
  "gene_name": "RB1-inducible coiled-coil protein 1"
}